{
  "gene_name": "A-kinase anchor protein 14",
  "gene": "UniProtKB:Q86UN6",
  "gene_symbol": "AKAP14",
  "term_id": "UNKNOWN:0002",
  "term_label": "Unknown biological process"
}